{
  "term_id": "GO:0005125",
  "gene_name": "Interleukin-3",
  "gene": "UniProtKB:P08700",
  "term_label": "cytokine activity",
  "gene_symbol": "IL3"
}